{
  "term_label": "protein-disulfide reductase [NAD(P)H] activity",
  "term_id": "GO:0047134",
  "gene_symbol": "TXNDC17",
  "gene_name": "Thioredoxin domain-containing protein 17",
  "gene": "UniProtKB:Q9BRA2"
}